{
  "term_label": "endoplasmic reticulum",
  "gene_symbol": "TMED9",
  "term_id": "GO:0005783",
  "gene": "UniProtKB:Q9BVK6",
  "gene_name": "Transmembrane emp24 domain-containing protein 9"
}